{
  "gene_symbol": "FBXL4",
  "gene": "UniProtKB:Q9UKA2",
  "term_label": "SCF-dependent proteasomal ubiquitin-dependent protein catabolic process",
  "gene_name": "F-box_LRR-repeat protein 4",
  "term_id": "GO:0031146"
}